{
  "term_label": "Unknown biological process",
  "gene": "UniProtKB:A0A1B0GUZ9",
  "gene_symbol": "A0A1B0GUZ9",
  "gene_name": "Uncharacterized protein",
  "term_id": "UNKNOWN:0002"
}